{
  "gene": "UniProtKB:P01258",
  "gene_symbol": "CALCA",
  "term_label": "extracellular space",
  "gene_name": "Calcitonin",
  "term_id": "GO:0005615"
}